mannose-ethanolamine phosphotransferase activity [GO:0051377] (molecular function) Definition: Catalysis of the transfer of ethanolamine phosphate to a mannose residue in the GPI lipid precursor. Relationships: is a type of phosphotransferase activity, for other substituted phosphate groups [GO:0016780] Also known as: ethanolamine phosphate transferase activity, phosphoethanolamine transferase activity, EtN-P transferase activity, addition of ethanolamine phosphate to mannose of GPI precursor References: PMID:15632136 Subtypes: GO:0051267